{
  "gene_name": "Inhibitor of growth protein 4",
  "gene_symbol": "ING4",
  "term_id": "GO:0006355",
  "term_label": "regulation of DNA-templated transcription",
  "gene": "UniProtKB:Q9UNL4"
}